{
  "term_id": "GO:0005739",
  "term_label": "mitochondrion",
  "gene_symbol": "MTCH1",
  "gene": "UniProtKB:Q9NZJ7",
  "gene_name": "Mitochondrial carrier homolog 1"
}